{
  "gene_name": "Uncharacterized protein C1orf232",
  "term_id": "UNKNOWN:0001",
  "gene": "UniProtKB:A0A0U1RR37",
  "gene_symbol": "C1orf232",
  "term_label": "Unknown molecular function"
}